INA complex [GO:1990524] (cellular component) Also known as: INAC Relationships: is a type of inner mitochondrial membrane protein complex [GO:0098800] Definition: A protein complex located in the inner membrane of mitochondria that is involved in the assembly of the peripheral (or stator) stalk of the mitochondrial proton-transporting ATP synthase (also known as the F1F0 ATP synthase). In budding yeast, this complex includes Ina22p and Ina17p. References: PMID:24942160 Sources: GOC:rn